mucociliary clearance [GO:0120197] (biological process) Definition: The respiratory system process driven by motile cilia on epithelial cells of the respiratory tract by which mucus and associated inhaled particles and pathogens trapped within it are moved out of the airways. Also known as: mucociliary transport, MCC, MCT Relationships: is a type of respiratory system process [GO:0003016]; is a type of epithelial cilium movement involved in extracellular fluid movement [GO:0003351] References: PMID:24119105, PMID:27864314 Sources: GOC:krc